{
  "gene_name": "Phosphatidylinositol-binding clathrin assembly protein",
  "gene": "UniProtKB:Q13492",
  "term_id": "GO:0000149",
  "term_label": "SNARE binding",
  "gene_symbol": "PICALM"
}